{
  "gene_symbol": "EMG1",
  "gene_name": "Ribosomal RNA small subunit methyltransferase NEP1",
  "term_label": "nucleus",
  "term_id": "GO:0005634",
  "gene": "UniProtKB:Q92979"
}